{
  "term_id": "UNKNOWN:0003",
  "gene_name": "Cytochrome P450 26A1",
  "gene_symbol": "CYP26A1",
  "gene": "UniProtKB:O43174",
  "term_label": "Unknown cellular component"
}